{
  "gene": "UniProtKB:Q9C0C4",
  "gene_symbol": "SEMA4C",
  "gene_name": "Semaphorin-4C",
  "term_label": "synaptic vesicle membrane",
  "term_id": "GO:0030672"
}